{
  "term_label": "mitotic metaphase chromosome alignment",
  "term_id": "GO:0007080",
  "gene_symbol": "CENPA",
  "gene_name": "Histone H3-like centromeric protein A",
  "gene": "UniProtKB:P49450"
}